{
  "gene_name": "Zinc finger protein neuro-d4",
  "gene": "UniProtKB:Q92782",
  "gene_symbol": "DPF1",
  "term_label": "nervous system development",
  "term_id": "GO:0007399"
}